establishment of episomal latency [GO:0075720] (biological process) Also known as: establishment of plasmid latency, establishment as a plasmid prophage Relationships: is a type of GO:0019043 Sources: GOC:jl Subtypes: establishment of latency as a circular episome [GO:0075529], establishment of latency as a linear episome [GO:0075530] Definition: A process by which a virus establishes a latent state within its host as an episome, where the viral genome remains silent in the cytoplasm or nucleus as a distinct genetic entity.